{
  "term_label": "cytoplasm",
  "term_id": "GO:0005737",
  "gene": "UniProtKB:A6NP61",
  "gene_name": "Protein ZAR1-like",
  "gene_symbol": "ZAR1L"
}